{
  "gene_symbol": "TMOD4",
  "gene_name": "Tropomodulin-4",
  "term_label": "myofibril",
  "gene": "UniProtKB:Q9NZQ9",
  "term_id": "GO:0030016"
}